{
  "gene_name": "Akirin-1",
  "gene_symbol": "AKIRIN1",
  "term_id": "GO:0010759",
  "term_label": "positive regulation of macrophage chemotaxis",
  "gene": "UniProtKB:Q9H9L7"
}